{
  "gene_symbol": "ARID2",
  "term_id": "GO:0005634",
  "term_label": "nucleus",
  "gene_name": "AT-rich interactive domain-containing protein 2",
  "gene": "UniProtKB:Q68CP9"
}